{
  "term_label": "nucleus",
  "term_id": "GO:0005634",
  "gene": "UniProtKB:Q9GZZ0",
  "gene_name": "Homeobox protein Hox-D1",
  "gene_symbol": "HOXD1"
}